{
  "gene": "UniProtKB:O14817",
  "term_id": "UNKNOWN:0001",
  "gene_symbol": "TSPAN4",
  "term_label": "Unknown molecular function",
  "gene_name": "Tetraspanin-4"
}